{
  "term_label": "phospholipase C-activating G protein-coupled receptor signaling pathway",
  "gene_symbol": "FPR1",
  "gene": "UniProtKB:P21462",
  "gene_name": "fMet-Leu-Phe receptor",
  "term_id": "GO:0007200"
}